{
  "gene_name": "Nucleoplasmin-3",
  "gene_symbol": "NPM3",
  "term_id": "GO:0005737",
  "gene": "UniProtKB:O75607",
  "term_label": "cytoplasm"
}